photomorphogenesis [GO:0009640] (biological process) Sources: GOC:lr Also known as: plant development in response to light Regulation: regulated by regulation of photomorphogenesis [GO:0010099]; RO_0002212 by negative regulation of photomorphogenesis [GO:0010100]; positively regulated by positive regulation of photomorphogenesis [GO:2000306] Definition: The control of plant growth, development, and differentiation by the duration and nature of light, independent of photosynthesis. Relationships: is a type of response to red or far red light [GO:0009639]; is a type of GO:0009791